{
  "gene_symbol": "HOXD1",
  "gene_name": "Homeobox protein Hox-D1",
  "term_id": "GO:0006357",
  "gene": "UniProtKB:Q9GZZ0",
  "term_label": "regulation of transcription by RNA polymerase II"
}